positive regulation of the force of heart contraction by chemical signal [GO:0003099] (biological process) Subtypes: positive regulation of the force of heart contraction by epinephrine-norepinephrine [GO:0001997], positive regulation of the force of heart contraction by epinephrine [GO:0003059], positive regulation of the force of heart contraction by norepinephrine [GO:0003061] Definition: Any process which increases the force of heart muscle contraction mediated by chemical signaling, hormonal, autocrine or paracrine. Also known as: positive regulation of the force of heart muscle contraction by chemical signal Sources: GOC:mtg_cardio Relationships: is a type of regulation of the force of heart contraction by chemical signal [GO:0003057]; is a type of GO:0045823